{
  "gene_name": "Putative activator of 90 kDa heat shock protein ATPase homolog 2",
  "gene_symbol": "AHSA2P",
  "term_id": "GO:0006457",
  "term_label": "protein folding",
  "gene": "UniProtKB:Q719I0"
}